spectrin [GO:0008091] (cellular component) Relationships: is a type of protein-containing complex [GO:0032991]; is part of GO:0030864 Sources: GOC:curators, ISBN:0815316194 Definition: Membrane associated dimeric protein (240 and 220 kDa) of erythrocytes. Forms a complex with ankyrin, actin and probably other components of the membrane cytoskeleton, so that there is a mesh of proteins underlying the plasma membrane, potentially restricting the lateral mobility of integral proteins.